L-fucose biosynthetic process [GO:0006005] (biological process) Definition: The chemical reactions and pathways resulting in the formation of L-fucose (6-deoxy-L-galactose). Also known as: L-fucose anabolism, L-fucose biosynthesis, L-fucose formation, L-fucose synthesis Sources: GOC:jl Relationships: is a type of fucose biosynthetic process [GO:0042353]; is a type of GO:0042354